{
  "gene_symbol": "SH2D2A",
  "gene": "UniProtKB:Q9NP31",
  "gene_name": "SH2 domain-containing protein 2A",
  "term_label": "protein-macromolecule adaptor activity",
  "term_id": "GO:0030674"
}